{
  "term_id": "GO:0000978",
  "term_label": "RNA polymerase II cis-regulatory region sequence-specific DNA binding",
  "gene_symbol": "ZNF584",
  "gene": "UniProtKB:Q8IVC4",
  "gene_name": "Zinc finger protein 584"
}